{
  "term_id": "GO:0015229",
  "gene_symbol": "SLC23A1",
  "term_label": "L-ascorbic acid transmembrane transporter activity",
  "gene_name": "Solute carrier family 23 member 1",
  "gene": "UniProtKB:Q9UHI7"
}